{
  "gene_name": "Leukocyte immunoglobulin-like receptor subfamily A member 6",
  "term_label": "plasma membrane",
  "gene_symbol": "LILRA6",
  "term_id": "GO:0005886",
  "gene": "UniProtKB:Q6PI73"
}